steroid metabolic process [GO:0008202] (biological process) Sources: ISBN:0198547684 Relationships: is a type of lipid metabolic process [GO:0006629] Regulation: RO_0002211 by GO:0019218; negatively regulated by negative regulation of steroid metabolic process [GO:0045939]; positively regulated by positive regulation of steroid metabolic process [GO:0045940] Also known as: steroid metabolism Definition: The chemical reactions and pathways involving steroids, compounds with a 1,2,cyclopentanoperhydrophenanthrene nucleus. Subtypes: steroid biosynthetic process [GO:0006694], steroid catabolic process [GO:0006706], bile acid metabolic process [GO:0008206], C21-steroid hormone metabolic process [GO:0008207], GO:0008209, estrogen metabolic process [GO:0008210], glucocorticoid metabolic process [GO:0008211], mineralocorticoid metabolic process [GO:0008212], GO:0016125, GO:0016131, vitamin D metabolic process [GO:0042359], ecdysteroid metabolic process [GO:0045455], brexanolone metabolic process [GO:0062173], (25S)-Delta(7)-dafachronate metabolic process [GO:1902056]